calcium-dependent outer dynein arm binding [GO:0120152] (molecular function) Relationships: is a type of GO:0048306 Definition: Binding to an outer dynein arm in the presence of calcium. References: PMID:18620543 Sources: GOC:krc